{
  "gene_symbol": "PKP1",
  "gene_name": "Plakophilin-1",
  "term_label": "nucleus",
  "gene": "UniProtKB:Q13835",
  "term_id": "GO:0005634"
}